{
  "gene_name": "Claudin-17",
  "term_id": "GO:0160184",
  "gene_symbol": "CLDN17",
  "term_label": "paracellular transport",
  "gene": "UniProtKB:P56750"
}